{
  "gene_symbol": "OXT",
  "term_id": "GO:0031855",
  "gene": "UniProtKB:P01178",
  "gene_name": "Oxytocin-neurophysin 1",
  "term_label": "oxytocin receptor binding"
}